{
  "gene": "UniProtKB:Q7Z406",
  "gene_name": "Myosin-14",
  "term_label": "mitotic cytokinesis",
  "gene_symbol": "MYH14",
  "term_id": "GO:0000281"
}